{
  "term_label": "regulation of transcription by RNA polymerase II",
  "gene_symbol": "RFX5",
  "gene": "UniProtKB:P48382",
  "gene_name": "DNA-binding protein RFX5",
  "term_id": "GO:0006357"
}